{
  "gene_name": "Synaptotagmin-like protein 5",
  "gene_symbol": "SYTL5",
  "term_id": "GO:0042043",
  "gene": "UniProtKB:Q8TDW5",
  "term_label": "neurexin family protein binding"
}